{
  "term_label": "DNA-binding transcription factor activity, RNA polymerase II-specific",
  "gene_symbol": "ZNF678",
  "gene": "UniProtKB:Q5SXM1",
  "term_id": "GO:0000981",
  "gene_name": "Zinc finger protein 678"
}